7-methylguanosine catabolic process [GO:0046119] (biological process) Relationships: is a type of 7-methylguanosine metabolic process [GO:0008618]; is_a guanosine-containing compound catabolic process [GO:1901069] Sources: ISBN:0198506732 Definition: The chemical reactions and pathways resulting in the breakdown of 7-methylguanosine, a modified nucleoside that forms a cap at the 5'-terminus of eukaryotic mRNA. Also known as: 7-methylguanosine breakdown, 7-methylguanosine catabolism, 7-methylguanosine degradation